{
  "gene_symbol": "DMD",
  "term_label": "neuron development",
  "gene_name": "Dystrophin",
  "term_id": "GO:0048666",
  "gene": "UniProtKB:P11532"
}